{
  "gene_name": "5'-AMP-activated protein kinase subunit gamma-2",
  "gene_symbol": "PRKAG2",
  "term_label": "cellular response to glucose starvation",
  "gene": "UniProtKB:Q9UGJ0",
  "term_id": "GO:0042149"
}